{
  "term_id": "UNKNOWN:0002",
  "gene": "UniProtKB:P18825",
  "gene_name": "Alpha-2C adrenergic receptor",
  "term_label": "Unknown biological process",
  "gene_symbol": "ADRA2C"
}